cellular response to vitamin B3 [GO:0071303] (biological process) Also known as: cellular response to niacin, cellular response to nicotinamide Relationships: is_a response to vitamin B3 [GO:0033552]; is_a cellular response to vitamin [GO:0071295] Definition: Any process that results in a change in state or activity of a cell (in terms of movement, secretion, enzyme production, gene expression, etc.) as a result of a vitamin B3 stimulus. Sources: GOC:mah